protein oxidation [GO:0018158] (biological process) Relationships: is a type of protein modification process [GO:0036211] Definition: The modification of a protein amino acid by oxidation. Regulation: RO_0002211 by regulation of protein oxidation [GO:1904806]; negatively regulated by negative regulation of protein oxidation [GO:1904807]; positively regulated by positive regulation of protein oxidation [GO:1904808] Subtypes: peptidyl-lysine oxidation [GO:0018057], peptidyl-cysteine oxidation [GO:0018171] Sources: GOC:ai Also known as: protein amino acid oxidation